{
  "term_id": "GO:0042761",
  "gene": "UniProtKB:Q9P035",
  "gene_name": "Very-long-chain (3R)-3-hydroxyacyl-CoA dehydratase 3",
  "gene_symbol": "HACD3",
  "term_label": "very long-chain fatty acid biosynthetic process"
}